{
  "gene_symbol": "PRKCG",
  "gene": "UniProtKB:P05129",
  "term_label": "Unknown cellular component",
  "gene_name": "Protein kinase C gamma type",
  "term_id": "UNKNOWN:0003"
}